{
  "gene_name": "Probable ATP-dependent RNA helicase DDX20",
  "term_label": "spliceosomal snRNP assembly",
  "gene_symbol": "DDX20",
  "term_id": "GO:0000387",
  "gene": "UniProtKB:Q9UHI6"
}